positive regulation of fever generation by prostaglandin secretion [GO:0100011] (biological process) Sources: GOC:cjm, GOC:obol Definition: Any prostaglandin secretion process that positively_regulates fever generation. Relationships: is a type of regulation of fever generation by prostaglandin secretion [GO:0100009]; RO_0002213 fever generation [GO:0001660]